{
  "term_id": "GO:0005762",
  "gene": "UniProtKB:Q9H2W6",
  "term_label": "mitochondrial large ribosomal subunit",
  "gene_symbol": "MRPL46",
  "gene_name": "Large ribosomal subunit protein mL46"
}